{
  "gene_name": "F-BAR domain only protein 2",
  "gene": "UniProtKB:Q0JRZ9",
  "term_id": "GO:0048268",
  "term_label": "clathrin coat assembly",
  "gene_symbol": "FCHO2"
}